{
  "term_label": "external side of plasma membrane",
  "gene": "UniProtKB:P30273",
  "gene_symbol": "FCER1G",
  "term_id": "GO:0009897",
  "gene_name": "High affinity immunoglobulin epsilon receptor subunit gamma"
}